{
  "gene": "UniProtKB:Q32M78",
  "gene_symbol": "ZNF699",
  "term_label": "RNA polymerase II cis-regulatory region sequence-specific DNA binding",
  "gene_name": "Zinc finger protein 699",
  "term_id": "GO:0000978"
}